{
  "gene_name": "Integrin alpha-M",
  "term_id": "GO:0038023",
  "gene": "UniProtKB:P11215",
  "gene_symbol": "ITGAM",
  "term_label": "signaling receptor activity"
}